{
  "gene": "UniProtKB:P19338",
  "gene_name": "Nucleolin",
  "term_label": "mRNA splicing, via spliceosome",
  "gene_symbol": "NCL",
  "term_id": "GO:0000398"
}